axial mesodermal cell fate specification [GO:0048327] (biological process) Relationships: is_a mesodermal cell fate specification [GO:0007501]; is part of axial mesodermal cell fate commitment [GO:0048322] Sources: GOC:dgh Regulation: regulated by regulation of axial mesodermal cell fate specification [GO:0048328]; negatively regulated by GO:0048329; positively regulated by positive regulation of axial mesodermal cell fate specification [GO:0048330] Also known as: axial mesoderm cell fate specification Definition: The process in which a cell becomes capable of differentiating autonomously into an axial mesoderm cell in an environment that is neutral with respect to the developmental pathway; upon specification, the cell fate can be reversed.